{
  "term_label": "plasma membrane",
  "gene_name": "Junctophilin-1",
  "gene_symbol": "JPH1",
  "term_id": "GO:0005886",
  "gene": "UniProtKB:Q9HDC5"
}